regulation of transforming growth factor beta2 production [GO:0032909] (biological process) Relationships: is a type of regulation of transforming growth factor beta production [GO:0071634]; regulates transforming growth factor beta2 production [GO:0032906] Also known as: regulation of TGF-B2 production, regulation of TGFB2 production, regulation of transforming growth factor-beta2 production Definition: Any process that modulates the frequency, rate, or extent of production of transforming growth factor-beta2. Subtypes: negative regulation of transforming growth factor beta2 production [GO:0032912], positive regulation of transforming growth factor beta2 production [GO:0032915] Sources: GOC:mah